{
  "gene": "UniProtKB:Q2MKA7",
  "term_label": "extracellular space",
  "gene_name": "R-spondin-1",
  "term_id": "GO:0005615",
  "gene_symbol": "RSPO1"
}